{
  "gene": "UniProtKB:P60153",
  "gene_symbol": "RNASE9",
  "term_id": "UNKNOWN:0001",
  "gene_name": "Inactive ribonuclease-like protein 9",
  "term_label": "Unknown molecular function"
}